{
  "gene_symbol": "SLC9A6",
  "term_id": "GO:0055037",
  "term_label": "recycling endosome",
  "gene_name": "Sodium_hydrogen exchanger 6",
  "gene": "UniProtKB:Q92581"
}